{
  "gene": "UniProtKB:P55957",
  "term_id": "GO:0005739",
  "term_label": "mitochondrion",
  "gene_symbol": "BID",
  "gene_name": "BH3-interacting domain death agonist"
}